{
  "gene_name": "CSC1-like protein 2",
  "gene": "UniProtKB:Q5T3F8",
  "term_id": "GO:0005886",
  "gene_symbol": "TMEM63B",
  "term_label": "plasma membrane"
}